negative regulation of photosynthesis, light reaction [GO:0043155] (biological process) Definition: Any process that stops, prevents, or reduces the frequency, rate or extent of the light-dependent reaction of photosynthesis. Also known as: down regulation of photosynthesis, light reaction, down-regulation of photosynthesis, light reaction, downregulation of photosynthesis, light reaction, inhibition of photosynthesis, light reaction Sources: GOC:jl Relationships: is_a regulation of photosynthesis, light reaction [GO:0042548]; is a type of negative regulation of photosynthesis [GO:1905156]; negatively regulates photosynthesis, light reaction [GO:0019684] Subtypes: photoinhibition [GO:0010205]